{
  "gene_name": "Chromodomain-helicase-DNA-binding protein 8",
  "term_label": "ATP hydrolysis activity",
  "gene_symbol": "CHD8",
  "term_id": "GO:0016887",
  "gene": "UniProtKB:Q9HCK8"
}